{
  "gene": "UniProtKB:Q8TCG2",
  "term_id": "GO:0004430",
  "gene_symbol": "PI4K2B",
  "term_label": "1-phosphatidylinositol 4-kinase activity",
  "gene_name": "Phosphatidylinositol 4-kinase type 2-beta"
}